{
  "term_label": "protein phosphatase type 1 complex",
  "gene": "UniProtKB:Q9UQK1",
  "gene_symbol": "PPP1R3C",
  "gene_name": "Protein phosphatase 1 regulatory subunit 3C",
  "term_id": "GO:0000164"
}